{
  "term_id": "GO:0042981",
  "term_label": "regulation of apoptotic process",
  "gene_name": "Angiotensinogen",
  "gene": "UniProtKB:P01019",
  "gene_symbol": "AGT"
}